{
  "gene": "UniProtKB:P14207",
  "gene_symbol": "FOLR2",
  "gene_name": "Folate receptor beta",
  "term_label": "sperm-egg recognition",
  "term_id": "GO:0035036"
}